Malpighian tubule morphogenesis [GO:0007443] (biological process) Note: See also the fly_anatomy.ontology term 'Malpighian tubule ; FBbt:00005786'. Definition: The process in which the anatomical structures of the Malpighian tubule are generated and organized. This process takes place entirely during the embryonic phase. A Malpighian tubule is a fine, thin-walled excretory tubule in insects which leads into the posterior part of the gut. Relationships: is a type of embryonic morphogenesis [GO:0048598]; is a type of renal tubule morphogenesis [GO:0061333]; is part of embryonic hindgut morphogenesis [GO:0048619]; is part of GO:0072002 Sources: GOC:bf, ISBN:0582227089